{
  "gene_symbol": "KAAG1",
  "gene": "UniProtKB:Q9UBP8",
  "term_label": "Unknown biological process",
  "term_id": "UNKNOWN:0002",
  "gene_name": "Kidney-associated antigen 1"
}